regulation of ribosome biogenesis [GO:0090069] (biological process) Definition: Any process that modulates the rate, frequency or extent of ribosome biogenesis. Ribosome biogenesis is the cellular process that results in the biosynthesis of constituent macromolecules, assembly, and arrangement of constituent parts of ribosome subunits. Subtypes: positive regulation of ribosome biogenesis [GO:0090070], negative regulation of ribosome biogenesis [GO:0090071] Sources: GOC:dph, GOC:tb Relationships: is a type of regulation of cellular component biogenesis [GO:0044087]; RO_0002211 ribosome biogenesis [GO:0042254]